{
  "gene_name": "Alpha-2-macroglobulin receptor-associated protein",
  "gene": "UniProtKB:P30533",
  "term_id": "GO:0048019",
  "gene_symbol": "LRPAP1",
  "term_label": "receptor antagonist activity"
}